thioredoxin-disulfide reductase complex [GO:1902515] (cellular component) Note: An example of this is thioredoxin reductase (TrxB) in E. coli [P0A9P4] in PMID:10947986. Relationships: is a type of oxidoreductase complex [GO:1990204] Definition: A protein complex which is capable of thioredoxin-disulfide reductase activity. References: PMID:10947986 Sources: GOC:TermGenie, GOC:bhm